{
  "term_label": "cytosol",
  "term_id": "GO:0005829",
  "gene_name": "Glycolipid transfer protein",
  "gene_symbol": "GLTP",
  "gene": "UniProtKB:Q9NZD2"
}